{
  "term_id": "GO:0060080",
  "gene_name": "Inhibitory synaptic factor 2A",
  "gene": "UniProtKB:Q6ZSG2",
  "gene_symbol": "INSYN2A",
  "term_label": "inhibitory postsynaptic potential"
}